negative regulation of intracellular mRNA localization [GO:1904581] (biological process) References: PMID:21471000 Sources: GOC:TermGenie, GO_REF:0000058 Also known as: down regulation of establishment and maintenance of intracellular RNA localization, down regulation of intracellular mRNA localisation, down regulation of intracellular mRNA localization, down regulation of mRNA localization, intracellular, down-regulation of establishment and maintenance of intracellular RNA localization, down-regulation of intracellular mRNA localisation, down-regulation of intracellular mRNA localization, down-regulation of mRNA localization, intracellular, downregulation of establishment and maintenance of intracellular RNA localization, downregulation of intracellular mRNA localisation, downregulation of intracellular mRNA localization, downregulation of mRNA localization, intracellular, negative regulation of establishment and maintenance of intracellular RNA localization, negative regulation of intracellular mRNA localisation, negative regulation of mRNA localization, intracellular, down regulation of intracellular mRNA positioning, down regulation of mRNA positioning, intracellular, down-regulation of intracellular mRNA positioning, down-regulation of mRNA positioning, intracellular, downregulation of intracellular mRNA positioning, downregulation of mRNA positioning, intracellular, inhibition of establishment and maintenance of intracellular RNA localization, inhibition of intracellular mRNA localisation, inhibition of intracellular mRNA localization, inhibition of intracellular mRNA positioning, inhibition of mRNA localization, intracellular, inhibition of mRNA positioning, intracellular, negative regulation of intracellular mRNA positioning, negative regulation of mRNA positioning, intracellular Relationships: is a type of negative regulation of biological process [GO:0048519]; is a type of regulation of intracellular mRNA localization [GO:1904580]; negatively regulates GO:0008298 Subtypes: negative regulation of bicoid mRNA localization [GO:0045853], negative regulation of pole plasm oskar mRNA localization [GO:0045855] Definition: Any process that stops, prevents or reduces the frequency, rate or extent of intracellular mRNA localization.